{
  "gene_name": "Synaptosomal-associated protein 25",
  "term_label": "exocytosis",
  "term_id": "GO:0006887",
  "gene_symbol": "SNAP25",
  "gene": "UniProtKB:P60880"
}